{
  "term_label": "JUN kinase binding",
  "gene_symbol": "MAPK8IP3",
  "gene": "UniProtKB:Q9UPT6",
  "gene_name": "C-Jun-amino-terminal kinase-interacting protein 3",
  "term_id": "GO:0008432"
}